{
  "gene_name": "Activin receptor type-1C",
  "gene_symbol": "ACVR1C",
  "term_id": "GO:0016361",
  "term_label": "activin receptor activity, type I",
  "gene": "UniProtKB:Q8NER5"
}